positive regulation of neutrophil apoptotic process [GO:0033031] (biological process) Sources: GOC:add, GOC:mtg_apoptosis Also known as: up regulation of neutrophil apoptosis, up-regulation of neutrophil apoptosis, upregulation of neutrophil apoptosis, activation of neutrophil apoptosis, positive regulation of neutrophil apoptosis, stimulation of neutrophil apoptosis Relationships: is a type of positive regulation of immune system process [GO:0002684]; is a type of regulation of neutrophil apoptotic process [GO:0033029]; is a type of positive regulation of myeloid cell apoptotic process [GO:0033034]; is a type of positive regulation of leukocyte apoptotic process [GO:2000108]; RO_0002213 neutrophil apoptotic process [GO:0001781] Definition: Any process that activates or increases the frequency, rate, or extent of neutrophil apoptotic process.